{
  "gene_symbol": "VPS16",
  "gene_name": "Vacuolar protein sorting-associated protein 16 homolog",
  "gene": "UniProtKB:Q9H269",
  "term_id": "GO:0030897",
  "term_label": "HOPS complex"
}